{
  "gene_name": "Integrin beta-5",
  "term_label": "integrin binding",
  "term_id": "GO:0005178",
  "gene_symbol": "ITGB5",
  "gene": "UniProtKB:P18084"
}